{
  "gene": "UniProtKB:Q8N456",
  "term_id": "GO:0035556",
  "gene_name": "Leucine-rich repeat-containing protein 18",
  "gene_symbol": "LRRC18",
  "term_label": "intracellular signal transduction"
}